non-intein-mediated protein splicing [GO:0030909] (biological process) Sources: GOC:mah Relationships: is_a GO:0030908 Definition: The post-translational removal of peptide sequences from within a protein sequence, by a process not involving inteins.